{
  "term_label": "cell surface",
  "gene_symbol": "KLRC4",
  "gene": "UniProtKB:O43908",
  "gene_name": "NKG2-F type II integral membrane protein",
  "term_id": "GO:0009986"
}